{
  "gene_name": "Polypyrimidine tract-binding protein 1",
  "gene": "UniProtKB:P26599",
  "term_label": "nucleus",
  "term_id": "GO:0005634",
  "gene_symbol": "PTBP1"
}